{
  "gene_symbol": "NKAIN2",
  "term_label": "Unknown cellular component",
  "gene": "UniProtKB:Q5VXU1",
  "term_id": "UNKNOWN:0003",
  "gene_name": "Sodium_potassium-transporting ATPase subunit beta-1-interacting protein 2"
}